mitochondrial leucyl-tRNA aminoacylation [GO:0070153] (biological process) Definition: The process of coupling leucine to leucyl-tRNA in a mitochondrion, catalyzed by leucyl-tRNA synthetase. In tRNA aminoacylation, the amino acid is first activated by linkage to AMP and then transferred to either the 2'- or the 3'-hydroxyl group of the 3'-adenosine residue of the tRNA. Sources: GOC:mah, GOC:mcc Relationships: is a type of GO:0006429; is a type of tRNA aminoacylation for mitochondrial protein translation [GO:0070127]